{
  "term_id": "GO:0031146",
  "gene": "UniProtKB:Q13309",
  "gene_symbol": "SKP2",
  "gene_name": "S-phase kinase-associated protein 2",
  "term_label": "SCF-dependent proteasomal ubiquitin-dependent protein catabolic process"
}